{
  "gene": "UniProtKB:Q969Z3",
  "gene_name": "Mitochondrial amidoxime reducing component 2",
  "term_label": "molybdopterin cofactor binding",
  "term_id": "GO:0043546",
  "gene_symbol": "MTARC2"
}